{
  "gene_symbol": "KICS2",
  "gene_name": "KICSTOR subunit 2",
  "term_id": "UNKNOWN:0001",
  "gene": "UniProtKB:Q96MD2",
  "term_label": "Unknown molecular function"
}